regulation of photosynthesis [GO:0010109] (biological process) Subtypes: regulation of photosynthesis, dark reaction [GO:0010110], regulation of photosynthesis, light reaction [GO:0042548], photosystem stoichiometry adjustment [GO:0080005], negative regulation of photosynthesis [GO:1905156], positive regulation of photosynthesis [GO:1905157] Definition: Any process that modulates the frequency, rate or extent of photosynthesis. Sources: GOC:sm Relationships: is_a GO:0019222; regulates photosynthesis [GO:0015979]